{
  "gene_symbol": "DTYMK",
  "gene": "UniProtKB:P23919",
  "term_label": "cytoplasm",
  "term_id": "GO:0005737",
  "gene_name": "Thymidylate kinase"
}